8-hydroxy-2'-deoxyguanosine DNA binding [GO:1905773] (molecular function) References: PMID:19734539 Sources: GOC:BHF, GOC:BHF_telomere, GOC:TermGenie, GOC:nc, GO_REF:0000067 Definition: Binding to 8-hydroxy-2'-deoxyguanosine an oxidized purine residue found in damaged DNA. Relationships: is a type of oxidized purine DNA binding [GO:0032357]